{
  "gene_name": "Acid-sensing ion channel 5",
  "term_id": "GO:0005886",
  "gene": "UniProtKB:Q9NY37",
  "term_label": "plasma membrane",
  "gene_symbol": "ASIC5"
}